cellular response to iron(III) ion [GO:0071283] (biological process) Also known as: cellular response to iron(III) Relationships: is a type of response to iron(III) ion [GO:0010041]; is a type of GO:0071281 Sources: GOC:mah Definition: Any process that results in a change in state or activity of a cell (in terms of movement, secretion, enzyme production, gene expression, etc.) as a result of an iron(III) ion stimulus.